{
  "gene": "UniProtKB:A8MYZ6",
  "gene_name": "Forkhead box protein O6",
  "gene_symbol": "FOXO6",
  "term_id": "GO:0000981",
  "term_label": "DNA-binding transcription factor activity, RNA polymerase II-specific"
}